{
  "gene": "UniProtKB:Q8NDB2",
  "term_id": "GO:0051898",
  "term_label": "negative regulation of phosphatidylinositol 3-kinase/protein kinase B signal transduction",
  "gene_symbol": "BANK1",
  "gene_name": "B-cell scaffold protein with ankyrin repeats"
}